{
  "gene_name": "Phenylalanine-4-hydroxylase",
  "gene": "UniProtKB:P00439",
  "term_label": "Unknown cellular component",
  "term_id": "UNKNOWN:0003",
  "gene_symbol": "PAH"
}